{
  "gene": "UniProtKB:O43704",
  "gene_name": "Sulfotransferase 1B1",
  "gene_symbol": "SULT1B1",
  "term_id": "GO:0004062",
  "term_label": "aryl sulfotransferase activity"
}